glutamate-cysteine ligase activity [GO:0004357] (molecular function) Regulation: regulated by glutamate-cysteine ligase regulator activity [GO:1990609] Also known as: L-glutamate:L-cysteine gamma-ligase (ADP-forming) activity, gamma-glutamyl-L-cysteine synthetase activity, gamma-glutamylcysteine synthetase activity, gamma-glutamylcysteinyl synthetase activity Definition: Catalysis of the reaction: L-cysteine + L-glutamate + ATP = L-gamma-glutamyl-L-cysteine + ADP + 2 H+ + phosphate. Sources: EC:6.3.2.2, RHEA:13285 Relationships: is a type of acid-amino acid ligase activity [GO:0016881]